{
  "gene_name": "Protein Tob2",
  "gene_symbol": "TOB2",
  "term_label": "regulation of gene expression",
  "gene": "UniProtKB:Q14106",
  "term_id": "GO:0010468"
}